{
  "gene": "UniProtKB:P08F94",
  "gene_symbol": "PKHD1",
  "term_label": "Unknown biological process",
  "gene_name": "Fibrocystin",
  "term_id": "UNKNOWN:0002"
}